{
  "term_label": "positive regulation of apoptotic signaling pathway",
  "gene_name": "Pro-cathepsin H",
  "term_id": "GO:2001235",
  "gene_symbol": "CTSH",
  "gene": "UniProtKB:P09668"
}